medulla oblongata formation [GO:0021580] (biological process) Relationships: is a type of anatomical structure formation involved in morphogenesis [GO:0048646]; is part of hindbrain formation [GO:0021576]; is part of medulla oblongata morphogenesis [GO:0021579] Also known as: medulla biosynthesis, medulla formation, myelencephalon biosynthesis, myelencephalon formation Definition: The process that gives rise to the medulla oblongata. This process pertains to the initial formation of a structure from unspecified parts. The medulla oblongata lies directly above the spinal cord and controls vital autonomic functions such as digestion, breathing and the control of heart rate. Sources: GOC:cls, GOC:dgh, GOC:dph, GOC:jid, GO_REF:0000021